riboflavin phosphotransferase activity [GO:0050257] (molecular function) Definition: Catalysis of the reaction: alpha-D-glucose 1-phosphate + riboflavin = D-glucose + FMN. Sources: EC:2.7.1.42, RHEA:20409 Also known as: D-glucose-1-phosphate:riboflavin 5'-phosphotransferase activity, G-1-P phosphotransferase activity, alpha-D-glucose-1-phosphate:riboflavin 5'-phosphotransferase activity, riboflavine phosphotransferase activity Relationships: is a type of kinase activity [GO:0016301]; is a type of GO:0016773